B cell homeostasis [GO:0001782] (biological process) Also known as: B lymphocyte homeostasis, B-cell homeostasis, B-lymphocyte homeostasis Subtypes: GO:0001922 Definition: The process of regulating the proliferation and elimination of B cells such that the total number of B cells within a whole or part of an organism is stable over time in the absence of an outside stimulus. Note: Note that this term represents the return of B cell levels to stable numbers following an immune response as well as the proliferation and elimination of B cells required to maintain stable numbers in the absence of an outside stimulus. References: PMID:12956429 Sources: GOC:add, ISBN:0781735149 Relationships: is a type of lymphocyte homeostasis [GO:0002260]